intracellular glucose homeostasis [GO:0001678] (biological process) Definition: A homeostatic process involved in the maintenance of a steady state level of glucose within a cell. Sources: GOC:dph, GOC:go_curators, GOC:tb Also known as: cell glucose homeostasis, cellular glucose homeostasis Relationships: is a type of GO:0042593; is a type of intracellular chemical homeostasis [GO:0055082] Subtypes: cellular response to glucose stimulus [GO:0071333]